{
  "gene": "UniProtKB:O75385",
  "term_label": "autophagosome assembly",
  "gene_symbol": "ULK1",
  "term_id": "GO:0000045",
  "gene_name": "Serine_threonine-protein kinase ULK1"
}